sexual sporulation [GO:0034293] (BP) Definition: The formation of spores derived from the products of meiosis. Sources: GOC:mah Also known as: meiotic spore formation, meiotic sporulation, sexual spore formation Relationships: is a type of developmental process involved in reproduction [GO:0003006]; is a type of GO:0043934; is part of GO:0051321 Subtypes: GO:0043935, plant-type sporogenesis [GO:0048236], sexual sporulation resulting in formation of a multicellular or syncytial spore [GO:0075285] Regulation: regulated by GO:0034306